{
  "term_id": "UNKNOWN:0002",
  "gene_symbol": "ANKEF1",
  "gene": "UniProtKB:Q9NU02",
  "gene_name": "Ankyrin repeat and EF-hand domain-containing protein 1",
  "term_label": "Unknown biological process"
}